lactate biosynthetic process from pyruvate [GO:0019244] (biological process) Sources: GOC:go_curators Relationships: is a type of GO:0006090; is a type of GO:0019249; has part lactate dehydrogenase activity [GO:0004457] Also known as: lactate anabolism from pyruvate, lactate formation from pyruvate, lactate synthesis from pyruvate, pyruvate fermentation to lactate Definition: The chemical reactions and pathways resulting in the formation of lactate from other compounds, including pyruvate. Subtypes: D(-)-lactate biosynthetic process from pyruvate [GO:0019245], GO:0019246